{
  "term_id": "GO:0042393",
  "gene_name": "Nucleosome assembly protein 1-like 3",
  "gene": "UniProtKB:Q99457",
  "term_label": "histone binding",
  "gene_symbol": "NAP1L3"
}